recombination within rDNA repeats [GO:0045458] (BP) Relationships: is a type of GO:0006310; is_a maintenance of rDNA [GO:0043007] Sources: GOC:go_curators, ISBN:0198506732 Definition: Genetic recombination within the DNA of the genes coding for ribosomal RNA. Note: Note that this term was reinstated from obsolete. Also known as: recombination within ribosomal DNA repeats